{
  "term_label": "actin cytoskeleton organization",
  "term_id": "GO:0030036",
  "gene_name": "Cytospin-A",
  "gene_symbol": "SPECC1L",
  "gene": "UniProtKB:Q69YQ0"
}